{
  "gene": "UniProtKB:Q6ZSB9",
  "term_label": "negative regulation of transcription by RNA polymerase II",
  "term_id": "GO:0000122",
  "gene_name": "Zinc finger and BTB domain-containing protein 49",
  "gene_symbol": "ZBTB49"
}